{
  "gene_name": "Integrin alpha-M",
  "gene_symbol": "ITGAM",
  "gene": "UniProtKB:P11215",
  "term_label": "integrin alphaM-beta2 complex",
  "term_id": "GO:0034688"
}